regulation of nucleotide metabolic process [GO:0006140] (biological process) Definition: Any process that modulates the frequency, rate or extent of the chemical reactions and pathways involving nucleotides. Sources: GOC:go_curators Also known as: regulation of nucleotide metabolism Relationships: is a type of regulation of nucleobase-containing compound metabolic process [GO:0019219]; is a type of regulation of phosphorus metabolic process [GO:0051174]; is a type of regulation of small molecule metabolic process [GO:0062012]; RO_0002211 GO:0009117 Subtypes: GO:0030808, regulation of nucleotide catabolic process [GO:0030811], GO:0045980, positive regulation of nucleotide metabolic process [GO:0045981], regulation of purine nucleotide metabolic process [GO:1900542]